myoblast fate commitment in head [GO:0014714] (biological process) Relationships: is a type of myoblast fate commitment [GO:0048625] Definition: The process, taking place in the head, whereby the developmental fate of a cell becomes restricted such that it will develop into a myoblast. A myoblast is a mononucleate cell type that, by fusion with other myoblasts, gives rise to the myotubes that eventually develop into skeletal muscle fibers. Sources: CL:0000056, GOC:mtg_muscle